{
  "gene_symbol": "SLBP",
  "term_label": "mRNA binding",
  "term_id": "GO:0003729",
  "gene_name": "Histone RNA hairpin-binding protein",
  "gene": "UniProtKB:Q14493"
}